{
  "term_label": "structural constituent of ribosome",
  "gene": "UniProtKB:P61353",
  "gene_name": "Large ribosomal subunit protein eL27",
  "term_id": "GO:0003735",
  "gene_symbol": "RPL27"
}